{
  "term_label": "Unknown biological process",
  "gene_symbol": "Q6Q795",
  "term_id": "UNKNOWN:0002",
  "gene": "UniProtKB:Q6Q795",
  "gene_name": "Putative viral protein-binding protein C1"
}